regulation of basophil degranulation [GO:1903581] (biological process) Relationships: is a type of regulation of myeloid leukocyte mediated immunity [GO:0002886]; is a type of regulation of leukocyte degranulation [GO:0043300]; is a type of regulation of immune response [GO:0050776]; regulates basophil degranulation [GO:0002561] References: PMID:10880837 Sources: GOC:TermGenie, GO_REF:0000058 Subtypes: negative regulation of basophil degranulation [GO:1903582], GO:1903583 Definition: Any process that modulates the frequency, rate or extent of basophil degranulation.